exosporium assembly [GO:0070499] (biological process) Sources: GOC:mah Definition: A process that is carried out at the cellular level which results in the formation of an exosporium, the outermost layer of a bacterial endospore. Also known as: exosporium formation Relationships: is a type of cellular component assembly [GO:0022607]; is a type of external encapsulating structure organization [GO:0045229]